{
  "gene": "UniProtKB:O15357",
  "term_label": "cytosol",
  "term_id": "GO:0005829",
  "gene_name": "Phosphatidylinositol 3,4,5-trisphosphate 5-phosphatase 2",
  "gene_symbol": "INPPL1"
}